{
  "term_label": "translation release factor complex",
  "term_id": "GO:0018444",
  "gene": "UniProtKB:P62495",
  "gene_symbol": "ETF1",
  "gene_name": "Eukaryotic peptide chain release factor subunit 1"
}